{
  "term_id": "UNKNOWN:0001",
  "gene": "UniProtKB:Q9Y5R8",
  "term_label": "Unknown molecular function",
  "gene_name": "Trafficking protein particle complex subunit 1",
  "gene_symbol": "TRAPPC1"
}